dorsal spinal cord interneuron anterior axon guidance [GO:0097380] (biological process) Relationships: is a type of GO:0033564; is a type of dorsal spinal cord interneuron axon guidance [GO:0097378] References: PMID:19545367 Sources: GOC:yaf Also known as: dorsal interneuron rostral axon projection Definition: The process in which the migration of an axon growth cone of a dorsal spinal cord interneuron is directed to a specific target site in the anterior direction along the anterior-posterior body axis in response to a combination of attractive and repulsive cues. The anterior-posterior axis is defined by a line that runs from the head or mouth of an organism to the tail or opposite end of the organism.